{
  "term_label": "intracellularly cGMP-activated cation channel activity",
  "gene": "UniProtKB:Q9NQW8",
  "gene_symbol": "CNGB3",
  "gene_name": "Cyclic nucleotide-gated cation channel beta-3",
  "term_id": "GO:0005223"
}